{
  "gene_symbol": "LIPG",
  "gene_name": "Endothelial lipase",
  "term_label": "fatty acid biosynthetic process",
  "gene": "UniProtKB:Q9Y5X9",
  "term_id": "GO:0006633"
}